{
  "gene_name": "Cortexin domain containing 2",
  "term_id": "UNKNOWN:0002",
  "term_label": "Unknown biological process",
  "gene_symbol": "CTXND2",
  "gene": "UniProtKB:A0A1B0GV90"
}